response to nutrient levels [GO:0031667] (BP) Subtypes: response to dietary excess [GO:0002021], sulfur utilization [GO:0006791], response to nutrient [GO:0007584], carbohydrate utilization [GO:0009758], carbon utilization [GO:0015976], nitrogen utilization [GO:0019740], GO:0031669, GO:0032094, GO:0042594, response to caloric restriction [GO:0061771], response to oxygen-glucose deprivation [GO:0090649] Definition: Any process that results in a change in state or activity of a cell or an organism (in terms of movement, secretion, enzyme production, gene expression, etc.) as a result of a stimulus reflecting the presence, absence, or concentration of nutrients. Sources: GOC:mah Regulation: regulated by regulation of response to nutrient levels [GO:0032107]; negatively regulated by negative regulation of response to nutrient levels [GO:0032108]; positively regulated by positive regulation of response to nutrient levels [GO:0032109] Relationships: is a type of response to stimulus [GO:0050896]